{
  "term_label": "fibroblast growth factor receptor binding",
  "gene": "UniProtKB:O43559",
  "gene_symbol": "FRS3",
  "term_id": "GO:0005104",
  "gene_name": "Fibroblast growth factor receptor substrate 3"
}